{
  "term_id": "GO:0031090",
  "gene_symbol": "VOPP1",
  "gene": "UniProtKB:Q96AW1",
  "term_label": "organelle membrane",
  "gene_name": "Vesicular, overexpressed in cancer, prosurvival protein 1"
}